{
  "gene": "UniProtKB:Q13404",
  "gene_symbol": "UBE2V1",
  "term_label": "DNA damage tolerance",
  "gene_name": "Ubiquitin-conjugating enzyme E2 variant 1",
  "term_id": "GO:0006301"
}